negative regulation of fumagillin biosynthetic process [GO:1902091] (BP) Definition: Any process that stops, prevents or reduces the frequency, rate or extent of fumagillin biosynthetic process. Also known as: down regulation of fumagillin anabolism, down regulation of fumagillin biosynthesis, down regulation of fumagillin biosynthetic process, down regulation of fumagillin formation, down regulation of fumagillin synthesis, down-regulation of fumagillin anabolism, down-regulation of fumagillin biosynthesis, down-regulation of fumagillin biosynthetic process, down-regulation of fumagillin formation, down-regulation of fumagillin synthesis, downregulation of fumagillin anabolism, downregulation of fumagillin biosynthesis, downregulation of fumagillin biosynthetic process, downregulation of fumagillin formation, downregulation of fumagillin synthesis, inhibition of fumagillin anabolism, inhibition of fumagillin biosynthesis, inhibition of fumagillin formation, inhibition of fumagillin synthesis, negative regulation of fumagillin anabolism, negative regulation of fumagillin biosynthesis, negative regulation of fumagillin formation, negative regulation of fumagillin synthesis, inhibition of fumagillin biosynthetic process References: PMID:23488861 Sources: GOC:TermGenie, GOC:di Relationships: is a type of negative regulation of biosynthetic process [GO:0009890]; is a type of GO:0062014; is a type of GO:1902090; negatively regulates fumagillin biosynthetic process [GO:1902086]